{
  "gene_name": "Carbohydrate sulfotransferase 4",
  "term_id": "GO:0006790",
  "term_label": "sulfur compound metabolic process",
  "gene": "UniProtKB:Q8NCG5",
  "gene_symbol": "CHST4"
}